{
  "gene_symbol": "FANCI",
  "gene": "UniProtKB:Q9NVI1",
  "term_label": "Unknown biological process",
  "term_id": "UNKNOWN:0002",
  "gene_name": "Fanconi anemia group I protein"
}